{
  "term_id": "GO:0004307",
  "gene_name": "Ethanolaminephosphotransferase 1",
  "gene": "UniProtKB:Q9C0D9",
  "gene_symbol": "SELENOI",
  "term_label": "ethanolaminephosphotransferase activity"
}